{
  "gene_name": "Suppressor of IKBKE 1",
  "term_label": "Unknown biological process",
  "gene": "UniProtKB:Q9BRV8",
  "term_id": "UNKNOWN:0002",
  "gene_symbol": "SIKE1"
}